{
  "gene": "UniProtKB:O75832",
  "gene_symbol": "PSMD10",
  "gene_name": "26S proteasome non-ATPase regulatory subunit 10",
  "term_id": "GO:0005634",
  "term_label": "nucleus"
}